feruloyl-CoA hydratase/lyase activity [GO:0050547] (molecular function) Relationships: is a type of aldehyde-lyase activity [GO:0016832] Definition: Catalysis of the reaction: (E)-feruloyl-CoA + H2O = acetyl-CoA + vanillin. Sources: RHEA:62412 Also known as: enoyl-CoA hydratase/aldolase activity, hydroxycinnamoyl-CoA hydratase lyase activity, vanillin synthase activity